regulation of inositol biosynthetic process [GO:1900088] (biological process) References: PMID:22307851 Sources: GOC:TermGenie Definition: Any process that modulates the frequency, rate or extent of inositol biosynthetic process. Subtypes: negative regulation of inositol biosynthetic process [GO:1900089], positive regulation of inositol biosynthetic process [GO:1900090] Also known as: regulation of inositol anabolism, regulation of inositol biosynthesis, regulation of inositol formation, regulation of inositol synthesis, regulation of vitamin Bh biosynthesis, regulation of vitamin Bh biosynthetic process, regulation of myo-inositol biosynthesis, regulation of myo-inositol biosynthetic process Relationships: is a type of regulation of alcohol biosynthetic process [GO:1902930]; regulates GO:0006021